{
  "gene_name": "AF4_FMR2 family member 2",
  "term_label": "nuclear speck",
  "gene_symbol": "AFF2",
  "gene": "UniProtKB:P51816",
  "term_id": "GO:0016607"
}